{
  "term_label": "Unknown biological process",
  "gene": "UniProtKB:Q9BZ98",
  "gene_symbol": "TTTY12",
  "term_id": "UNKNOWN:0002",
  "gene_name": "Putative transcript Y 12 protein"
}